{
  "gene": "UniProtKB:O60518",
  "gene_name": "Ran-binding protein 6",
  "gene_symbol": "RANBP6",
  "term_label": "protein import into nucleus",
  "term_id": "GO:0006606"
}